negative regulation of monoatomic ion transmembrane transport [GO:0034766] (biological process) Relationships: is a type of negative regulation of transmembrane transport [GO:0034763]; is a type of regulation of monoatomic ion transmembrane transport [GO:0034765]; is a type of GO:0043271; negatively regulates GO:0034220 Also known as: negative regulation of ion transmembrane transport, down regulation of transmembrane ion transport, down-regulation of transmembrane ion transport, downregulation of transmembrane ion transport, negative regulation of ion membrane transport, negative regulation of transmembrane ion transport, inhibition of transmembrane ion transport Subtypes: negative regulation of ion transmembrane transporter activity [GO:0032413], negative regulation of anion transmembrane transport [GO:1903960], GO:1904063 Definition: Any process that stops, prevents, or reduces the frequency, rate or extent of the directed movement of ions from one side of a membrane to the other. Sources: GOC:mah